{
  "gene": "UniProtKB:P32881",
  "gene_symbol": "IFNA8",
  "term_id": "GO:0005132",
  "gene_name": "Interferon alpha-8",
  "term_label": "type I interferon receptor binding"
}